{
  "term_label": "Golgi apparatus",
  "gene_symbol": "GALNT14",
  "gene_name": "Polypeptide N-acetylgalactosaminyltransferase 14",
  "gene": "UniProtKB:Q96FL9",
  "term_id": "GO:0005794"
}